{
  "gene": "UniProtKB:Q9BQ75",
  "gene_symbol": "CMSS1",
  "term_label": "Unknown molecular function",
  "term_id": "UNKNOWN:0001",
  "gene_name": "Protein CMSS1"
}